{
  "term_id": "GO:0051552",
  "term_label": "flavone metabolic process",
  "gene": "UniProtKB:P22309",
  "gene_symbol": "UGT1A1",
  "gene_name": "UDP-glucuronosyltransferase 1A1"
}